{
  "term_id": "GO:0031467",
  "gene": "UniProtKB:Q8N3Y1",
  "gene_symbol": "FBXW8",
  "term_label": "Cul7-RING ubiquitin ligase complex",
  "gene_name": "F-box_WD repeat-containing protein 8"
}